{
  "gene_symbol": "LRG1",
  "term_label": "positive regulation of angiogenesis",
  "term_id": "GO:0045766",
  "gene": "UniProtKB:P02750",
  "gene_name": "Leucine-rich alpha-2-glycoprotein"
}